ensheathing process [GO:1990015] (cellular component) Relationships: is a type of cellular anatomical structure [GO:0110165] Definition: A cell projection (often from glial cells such as Schwann cells) that surrounds an unmyelinated axon or cell soma. Subtypes: GO:0097453 Also known as: ensheathing process of Schwann cell Sources: NIF_Subcellular:sao1376748732